striated muscle tissue development [GO:0014706] (biological process) Sources: CL:0000737, GOC:dph, GOC:mtg_muscle Subtypes: pulmonary myocardium development [GO:0003350], GO:0007519, GO:0048738 Definition: The process whose specific outcome is the progression of a striated muscle over time, from its formation to the mature structure. Striated muscle contain fibers that are divided by transverse bands into striations, and cardiac and skeletal muscle are types of striated muscle. Skeletal muscle myoblasts fuse to form myotubes and eventually multinucleated muscle fibers. The fusion of cardiac cells is very rare and can only form binucleate cells. Regulation: regulated by regulation of striated muscle tissue development [GO:0016202]; negatively regulated by negative regulation of striated muscle tissue development [GO:0045843]; positively regulated by GO:0045844 Relationships: is a type of GO:0060537